{
  "gene_symbol": "WSB1",
  "gene": "UniProtKB:Q9Y6I7",
  "term_id": "UNKNOWN:0001",
  "gene_name": "WD repeat and SOCS box-containing protein 1",
  "term_label": "Unknown molecular function"
}